{
  "term_label": "photoreceptor inner segment",
  "term_id": "GO:0001917",
  "gene_symbol": "GUCA1A",
  "gene_name": "Guanylyl cyclase-activating protein 1",
  "gene": "UniProtKB:P43080"
}